regulation of compound eye retinal cell programmed cell death [GO:0046669] (biological process) Definition: Any process that modulates the frequency, rate or extent of programmed cell death that occurs in the compound eye retina. Sources: GOC:ai Also known as: regulation of retinal cell programmed cell death Relationships: is a type of regulation of retinal cell programmed cell death [GO:0046668]; regulates compound eye retinal cell programmed cell death [GO:0046667] Subtypes: positive regulation of compound eye retinal cell programmed cell death [GO:0046672], negative regulation of compound eye retinal cell programmed cell death [GO:0046673]